{
  "term_label": "mitophagy",
  "gene_name": "Gamma-aminobutyric acid receptor-associated protein-like 3",
  "term_id": "GO:0000423",
  "gene": "UniProtKB:Q9BY60",
  "gene_symbol": "GABARAPL3"
}